{
  "gene": "UniProtKB:Q96CN5",
  "term_label": "plasma membrane",
  "term_id": "GO:0005886",
  "gene_symbol": "LRRC45",
  "gene_name": "Leucine-rich repeat-containing protein 45"
}